{
  "term_id": "GO:0005829",
  "gene_name": "Segment polarity protein dishevelled homolog DVL-1",
  "gene": "UniProtKB:O14640",
  "term_label": "cytosol",
  "gene_symbol": "DVL1"
}